{
  "term_label": "endocytosis",
  "gene": "UniProtKB:Q9H201",
  "term_id": "GO:0006897",
  "gene_symbol": "EPN3",
  "gene_name": "Epsin-3"
}